{
  "gene_symbol": "LCP1",
  "term_label": "cytoplasm",
  "gene_name": "Plastin-2",
  "gene": "UniProtKB:P13796",
  "term_id": "GO:0005737"
}